negative regulation of membrane repolarization during ventricular cardiac muscle cell action potential [GO:1905025] (biological process) Also known as: down regulation of membrane repolarization during ventricular cardiac muscle cell action potential, down-regulation of membrane repolarization during ventricular cardiac muscle cell action potential, downregulation of membrane repolarization during ventricular cardiac muscle cell action potential, inhibition of membrane repolarization during ventricular cardiac muscle cell action potential, down regulation of electrocardiogram T wave, down regulation of regulation of ventricular cardiac muscle repolarization, down regulation of ventricular repolarization, down-regulation of electrocardiogram T wave, down-regulation of regulation of ventricular cardiac muscle repolarization, down-regulation of ventricular repolarization, downregulation of electrocardiogram T wave, downregulation of regulation of ventricular cardiac muscle repolarization, downregulation of ventricular repolarization, inhibition of electrocardiogram T wave, inhibition of regulation of ventricular cardiac muscle repolarization, inhibition of ventricular repolarization, negative regulation of electrocardiogram T wave, negative regulation of regulation of ventricular cardiac muscle repolarization, negative regulation of ventricular repolarization Relationships: is a type of GO:1905024; is a type of GO:1905032; negatively regulates membrane repolarization during ventricular cardiac muscle cell action potential [GO:0098915] Definition: Any process that stops, prevents or reduces the frequency, rate or extent of membrane repolarization during ventricular cardiac muscle cell action potential. References: PMID:19893015 Sources: GOC:BHF, GOC:BHF_miRNA, GOC:TermGenie, GOC:mtg_cardiac_conduct_nov11, GOC:rph